{
  "gene": "UniProtKB:Q15643",
  "gene_name": "Thyroid receptor-interacting protein 11",
  "term_id": "GO:0031267",
  "term_label": "small GTPase binding",
  "gene_symbol": "TRIP11"
}